structural constituent of proteasome [GO:0140756] (molecular function) Definition: The action of a molecule that contributes to the structural integrity of the proteasome. References: PMID:10500111, PMID:28525752, PMID:28583440, PMID:29652515 Relationships: is a type of structural molecule activity [GO:0005198]; occurs in GO:0000502